morphine metabolic process [GO:0071272] (biological process) Subtypes: GO:0071273, morphine biosynthetic process [GO:0097295] Also known as: morphine metabolism Definition: The chemical reactions and pathways involving morphine, 17-methyl-7,8-didehydro-4,5alpha-epoxymorphinan-3,6alpha-diol. Morphine is a highly potent opiate analgesic psychoactive drug obtained form the opium poppy, Papaver somniferum. Sources: GOC:mah Relationships: is a type of GO:0033076